{
  "gene_name": "DNA-binding protein inhibitor ID-4",
  "gene": "UniProtKB:P47928",
  "term_id": "GO:0030182",
  "term_label": "neuron differentiation",
  "gene_symbol": "ID4"
}